{
  "term_id": "GO:0010571",
  "gene_name": "Protein DBF4 homolog B",
  "gene": "UniProtKB:Q8NFT6",
  "gene_symbol": "DBF4B",
  "term_label": "positive regulation of nuclear cell cycle DNA replication"
}